{
  "term_id": "GO:0035517",
  "term_label": "PR-DUB complex",
  "gene_name": "Putative Polycomb group protein ASXL2",
  "gene": "UniProtKB:Q76L83",
  "gene_symbol": "ASXL2"
}